{
  "term_id": "UNKNOWN:0001",
  "gene_name": "FK506-binding protein 15",
  "term_label": "Unknown molecular function",
  "gene_symbol": "FKBP15",
  "gene": "UniProtKB:Q5T1M5"
}